{
  "gene_symbol": "TSPY1",
  "term_label": "Unknown biological process",
  "gene": "UniProtKB:Q01534",
  "term_id": "UNKNOWN:0002",
  "gene_name": "Testis-specific Y-encoded protein 1"
}